{
  "gene": "UniProtKB:Q96KQ7",
  "term_label": "epigenetic regulation of gene expression",
  "gene_name": "Histone-lysine N-methyltransferase EHMT2",
  "term_id": "GO:0040029",
  "gene_symbol": "EHMT2"
}